{
  "term_id": "GO:0045944",
  "gene_name": "Transcriptional activator Myb",
  "gene": "UniProtKB:P10242",
  "term_label": "positive regulation of transcription by RNA polymerase II",
  "gene_symbol": "MYB"
}